negative regulation of cellular response to testosterone stimulus [GO:2000655] (biological process) Sources: GOC:BHF Relationships: is a type of negative regulation of cellular process [GO:0048523]; is a type of negative regulation of response to stimulus [GO:0048585]; is a type of regulation of cellular response to testosterone stimulus [GO:2000654]; negatively regulates cellular response to testosterone stimulus [GO:0071394] Definition: Any process that stops, prevents or reduces the frequency, rate or extent of cellular response to testosterone stimulus.